{
  "gene_symbol": "PRR33",
  "gene": "UniProtKB:A8MZF0",
  "gene_name": "Proline-rich protein 33",
  "term_label": "Unknown molecular function",
  "term_id": "UNKNOWN:0001"
}